{
  "term_id": "GO:0055085",
  "gene": "UniProtKB:Q03519",
  "gene_name": "Antigen peptide transporter 2",
  "gene_symbol": "TAP2",
  "term_label": "transmembrane transport"
}